{
  "gene_name": "Sorting nexin-17",
  "gene_symbol": "SNX17",
  "term_id": "GO:0032456",
  "term_label": "endocytic recycling",
  "gene": "UniProtKB:Q15036"
}